{
  "term_label": "retrograde transport, endosome to Golgi",
  "gene_name": "WASH complex subunit 2A",
  "term_id": "GO:0042147",
  "gene_symbol": "WASHC2A",
  "gene": "UniProtKB:Q641Q2"
}